regulation of TORC1 signaling [GO:1903432] (biological process) Also known as: regulation of TORC1 signal transduction Definition: Any process that modulates the frequency, rate or extent of TORC1 signaling. Subtypes: negative regulation of TORC1 signaling [GO:1904262], positive regulation of TORC1 signaling [GO:1904263] Relationships: is a type of regulation of TOR signaling [GO:0032006]; regulates TORC1 signaling [GO:0038202] Sources: GOC:TermGenie, GO_REF:0000058